{
  "gene_symbol": "KLF17",
  "gene": "UniProtKB:Q5JT82",
  "term_id": "GO:0000981",
  "term_label": "DNA-binding transcription factor activity, RNA polymerase II-specific",
  "gene_name": "Krueppel-like factor 17"
}